{
  "gene": "UniProtKB:Q8NDV7",
  "term_id": "GO:0000932",
  "gene_name": "Trinucleotide repeat-containing gene 6A protein",
  "gene_symbol": "TNRC6A",
  "term_label": "P-body"
}